cellular response to salt stress [GO:0071472] (biological process) Definition: Any process that results in a change in state or activity of a cell (in terms of movement, secretion, enzyme production, gene expression, etc.) as a result of a stimulus indicating an increase or decrease in the concentration of salt (particularly but not exclusively sodium and chloride ions) in the environment. Relationships: is a type of response to salt stress [GO:0009651]; is a type of cellular response to osmotic stress [GO:0071470] Subtypes: GO:0071473, cellular hyperosmotic salinity response [GO:0071475], cellular hypotonic salinity response [GO:0071477] Sources: GOC:mah Also known as: cellular response to ionic osmotic stress, cellular salinity response